{
  "gene": "UniProtKB:O60676",
  "term_id": "UNKNOWN:0001",
  "gene_name": "Cystatin-8",
  "term_label": "Unknown molecular function",
  "gene_symbol": "CST8"
}